{
  "term_label": "double-stranded DNA binding",
  "term_id": "GO:0003690",
  "gene": "UniProtKB:Q9NUD5",
  "gene_name": "Zinc finger CCHC domain-containing protein 3",
  "gene_symbol": "ZCCHC3"
}